{
  "gene_symbol": "PAXIP1",
  "term_label": "nucleus",
  "term_id": "GO:0005634",
  "gene_name": "PAX-interacting protein 1",
  "gene": "UniProtKB:Q6ZW49"
}